{
  "gene_symbol": "ARMCX3",
  "gene": "UniProtKB:Q9UH62",
  "gene_name": "Armadillo repeat-containing X-linked protein 3",
  "term_label": "mitochondrion",
  "term_id": "GO:0005739"
}